{
  "gene": "UniProtKB:Q8TDY4",
  "term_id": "GO:0016477",
  "term_label": "cell migration",
  "gene_symbol": "ASAP3",
  "gene_name": "Arf-GAP with SH3 domain, ANK repeat and PH domain-containing protein 3"
}